mineralocorticoid biosynthetic process [GO:0006705] (biological process) Definition: The chemical reactions and pathways resulting in the formation of mineralocorticoids, hormonal C21 corticosteroids synthesized from cholesterol. Sources: ISBN:0198506732 Also known as: mineralocorticoid anabolism, mineralocorticoid biosynthesis, mineralocorticoid formation, mineralocorticoid synthesis Relationships: is a type of mineralocorticoid metabolic process [GO:0008212]; is_a hormone biosynthetic process [GO:0042446]; is a type of steroid hormone biosynthetic process [GO:0120178] Subtypes: GO:0032342